{
  "term_label": "Unknown molecular function",
  "gene_symbol": "TEX264",
  "gene": "UniProtKB:Q9Y6I9",
  "term_id": "UNKNOWN:0001",
  "gene_name": "Testis-expressed protein 264"
}